{
  "gene_name": "Neuronal pentraxin receptor",
  "gene": "UniProtKB:O95502",
  "gene_symbol": "NPTXR",
  "term_label": "Unknown molecular function",
  "term_id": "UNKNOWN:0001"
}